{
  "gene_symbol": "RBM7",
  "gene_name": "RNA-binding protein 7",
  "term_label": "regulation of alternative mRNA splicing, via spliceosome",
  "term_id": "GO:0000381",
  "gene": "UniProtKB:Q9Y580"
}